{
  "gene_name": "T cell receptor alpha joining 42",
  "term_label": "Unknown molecular function",
  "term_id": "UNKNOWN:0001",
  "gene_symbol": "TRAJ42",
  "gene": "UniProtKB:A0A075B6Y9"
}